negative regulation of ubiquitin-dependent endocytosis [GO:2000396] (biological process) Sources: GOC:mah Also known as: negative regulation of ubiquitin-mediated endocytosis Relationships: is a type of GO:0045806; is a type of GO:0051224; is a type of regulation of ubiquitin-dependent endocytosis [GO:2000395]; negatively regulates ubiquitin-dependent endocytosis [GO:0070086] Definition: Any process that stops, prevents or reduces the frequency, rate or extent of ubiquitin-dependent endocytosis.